{
  "term_id": "UNKNOWN:0002",
  "gene_name": "Transmembrane protein 263",
  "gene": "UniProtKB:Q8WUH6",
  "term_label": "Unknown biological process",
  "gene_symbol": "TMEM263"
}